{
  "gene_name": "Olfactory receptor 4K14",
  "term_label": "olfactory receptor activity",
  "term_id": "GO:0004984",
  "gene": "UniProtKB:Q8NGD5",
  "gene_symbol": "OR4K14"
}